{
  "gene": "UniProtKB:P68871",
  "term_label": "haptoglobin-hemoglobin complex",
  "term_id": "GO:0031838",
  "gene_symbol": "HBB",
  "gene_name": "Hemoglobin subunit beta"
}